{
  "term_id": "UNKNOWN:0001",
  "term_label": "Unknown molecular function",
  "gene": "UniProtKB:O75691",
  "gene_symbol": "UTP20",
  "gene_name": "Small subunit processome component 20 homolog"
}